pyruvate transmembrane transport [GO:1901475] (biological process) Subtypes: plasma membrane pyruvate transport [GO:0006849], pyruvate import into mitochondria [GO:0006850] Definition: The directed movement of pyruvate across a membrane. Also known as: pyruvate membrane transport Relationships: is a type of pyruvate transport [GO:0006848]; is a type of carboxylic acid transmembrane transport [GO:1905039] Sources: GOC:TermGenie Note: Note that this term is not intended for use in annotating lateral movement within membranes.